{
  "term_id": "UNKNOWN:0001",
  "gene": "UniProtKB:Q4VC05",
  "gene_symbol": "BCL7A",
  "term_label": "Unknown molecular function",
  "gene_name": "B-cell CLL_lymphoma 7 protein family member A"
}